negative regulation of anterograde dense core granule transport [GO:1901952] (biological process) Definition: Any process that stops, prevents or reduces the frequency, rate or extent of anterograde dense core granule transport. References: PMID:23358451 Sources: GOC:TermGenie, GOC:kmv Also known as: down regulation of anterograde dense core granule transport, down-regulation of anterograde dense core granule transport, downregulation of anterograde dense core granule transport, inhibition of anterograde dense core granule transport Relationships: is a type of negative regulation of vesicle transport along microtubule [GO:1901609]; is a type of regulation of anterograde dense core granule transport [GO:1901951]; is a type of GO:1904810; RO_0002212 GO:1990048